{
  "gene": "UniProtKB:Q05481",
  "term_id": "GO:0006357",
  "term_label": "regulation of transcription by RNA polymerase II",
  "gene_symbol": "ZNF91",
  "gene_name": "Zinc finger protein 91"
}